{
  "gene": "UniProtKB:P04808",
  "gene_symbol": "RLN1",
  "term_id": "UNKNOWN:0001",
  "term_label": "Unknown molecular function",
  "gene_name": "Prorelaxin H1"
}